{
  "term_id": "GO:0030214",
  "gene_name": "Hyaluronidase-1",
  "gene": "UniProtKB:Q12794",
  "term_label": "hyaluronan catabolic process",
  "gene_symbol": "HYAL1"
}